endodermal cell fate specification [GO:0001714] (BP) Sources: GOC:go_curators Also known as: endoderm cell fate specification Definition: The cell fate determination process that results in a cell becoming capable of differentiating autonomously into an endoderm cell in an environment that is neutral with respect to the developmental pathway; upon specification, the cell fate can be reversed. Relationships: is a type of cell fate specification [GO:0001708]; is part of endodermal cell fate commitment [GO:0001711] Regulation: regulated by regulation of endodermal cell fate specification [GO:0042663]; negatively regulated by negative regulation of endodermal cell fate specification [GO:0042664]